{
  "term_label": "DNA-binding transcription factor activity, RNA polymerase II-specific",
  "gene": "UniProtKB:O60393",
  "gene_symbol": "NOBOX",
  "gene_name": "Homeobox protein NOBOX",
  "term_id": "GO:0000981"
}